{
  "gene_symbol": "ODAD3",
  "gene": "UniProtKB:A5D8V7",
  "term_id": "GO:0036158",
  "term_label": "outer dynein arm assembly",
  "gene_name": "Outer dynein arm-docking complex subunit 3"
}